hydrogen generation via biophotolysis [GO:0044817] (biological process) Definition: The production of hydrogen which results from the dissociation by light of water into molecular hydrogen and oxygen. This process is observed in cyanobacteria and microalgae. Also known as: hydrogen biosynthesis via biophotolysis References: PMID:20395274, PMID:20692761 Sources: GOC:mengo_curators Relationships: is a type of hydrogen biosynthetic process [GO:1902422]